{
  "term_label": "membrane",
  "term_id": "GO:0016020",
  "gene_name": "Scavenger receptor class F member 1",
  "gene": "UniProtKB:Q14162",
  "gene_symbol": "SCARF1"
}